methanol catabolic process [GO:0046170] (biological process) Sources: GOC:ai Relationships: is a type of methanol metabolic process [GO:0015945]; is a type of primary alcohol catabolic process [GO:0034310] Also known as: methanol breakdown, methanol catabolism, methanol degradation Definition: The chemical reactions and pathways resulting in the breakdown of methanol, CH3-OH, a colorless, flammable, mobile, poisonous liquid, widely used as a solvent.